{
  "term_id": "UNKNOWN:0003",
  "term_label": "Unknown cellular component",
  "gene_symbol": "PRR23A",
  "gene_name": "Proline-rich protein 23A",
  "gene": "UniProtKB:A6NEV1"
}